{
  "term_id": "GO:0006812",
  "gene": "UniProtKB:Q96RD6",
  "gene_name": "Pannexin-2",
  "term_label": "monoatomic cation transport",
  "gene_symbol": "PANX2"
}